{
  "gene_name": "Coiled-coil domain-containing protein 188",
  "term_id": "UNKNOWN:0003",
  "gene_symbol": "CCDC188",
  "term_label": "Unknown cellular component",
  "gene": "UniProtKB:H7C350"
}